{
  "gene_name": "Pejvakin",
  "term_id": "GO:0007605",
  "gene_symbol": "PJVK",
  "gene": "UniProtKB:Q0ZLH3",
  "term_label": "sensory perception of sound"
}